{
  "gene_symbol": "HSD17B6",
  "term_id": "GO:0008202",
  "gene_name": "17-beta-hydroxysteroid dehydrogenase type 6",
  "term_label": "steroid metabolic process",
  "gene": "UniProtKB:O14756"
}